T-helper 2 cell differentiation [GO:0045064] (biological process) Regulation: RO_0002211 by regulation of T-helper 2 cell differentiation [GO:0045628]; negatively regulated by GO:0045629; positively regulated by positive regulation of T-helper 2 cell differentiation [GO:0045630] Definition: The process in which a relatively unspecialized T cell acquires specialized features of a T-helper 2 (Th2) cell. A Th2 cell is a CD4-positive, alpha-beta T cell that has the phenotype GATA-3-positive and produces interleukin-4. Sources: CL:0000546, GOC:ebc Note: Note that immunologists typically use the word 'development' to refer to cells of B or T cell lineages undergoing the process that GO describes as 'cell differentiation'. Relationships: is a type of T-helper cell differentiation [GO:0042093]; is part of type 2 immune response [GO:0042092] Also known as: T-helper 2 cell development